{
  "term_label": "axon terminus",
  "gene": "UniProtKB:Q03721",
  "term_id": "GO:0043679",
  "gene_name": "Potassium voltage-gated channel subfamily C member 4",
  "gene_symbol": "KCNC4"
}